{
  "term_label": "Unknown molecular function",
  "gene_symbol": "TTC39B",
  "gene": "UniProtKB:Q5VTQ0",
  "gene_name": "Tetratricopeptide repeat protein 39B",
  "term_id": "UNKNOWN:0001"
}